{
  "gene_name": "Neuronal growth regulator 1",
  "gene": "UniProtKB:Q7Z3B1",
  "term_label": "Unknown molecular function",
  "term_id": "UNKNOWN:0001",
  "gene_symbol": "NEGR1"
}